{
  "gene_name": "Potassium voltage-gated channel subfamily A member 5",
  "gene_symbol": "KCNA5",
  "gene": "UniProtKB:P22460",
  "term_id": "GO:0071805",
  "term_label": "potassium ion transmembrane transport"
}